{
  "gene_symbol": "PRND",
  "gene_name": "Prion-like protein doppel",
  "term_id": "GO:0005507",
  "term_label": "copper ion binding",
  "gene": "UniProtKB:Q9UKY0"
}